skeletal muscle satellite cell activation [GO:0014719] (biological process) References: PMID:23303905 Sources: GOC:mtg_muscle Definition: The change of a skeletal muscle satellite cell from a mitotically quiescent to a mitotically active state following exposure to some activating factor such as a cellular or soluble ligand. In adult muscle, satellite cells become activated to divide and differentiate in response to muscle damage. Relationships: is a type of GO:0001775 Subtypes: satellite cell activation involved in skeletal muscle regeneration [GO:0014901]